{
  "term_id": "GO:0070034",
  "gene_name": "Telomerase-binding protein EST1A",
  "gene": "UniProtKB:Q86US8",
  "term_label": "telomerase RNA binding",
  "gene_symbol": "SMG6"
}